negative regulation of toll-like receptor 8 signaling pathway [GO:0034160] (biological process) Relationships: is a type of regulation of toll-like receptor 8 signaling pathway [GO:0034159]; is a type of GO:0039532; negatively regulates toll-like receptor 8 signaling pathway [GO:0034158] Definition: Any process that stops, prevents, or reduces the frequency, rate, or extent of toll-like receptor 8 signaling pathway. Also known as: negative regulation of TLR8 signaling pathway, negative regulation of toll-like receptor 8 signalling pathway References: PMID:16551253, PMID:17328678 Sources: GOC:add